positive regulation of nurse cell apoptotic process [GO:0045850] (biological process) Definition: Any process that activates or increases the frequency, rate or extent of nurse cell apoptotic process. Relationships: is a type of regulation of nurse cell apoptotic process [GO:0045477]; is a type of positive regulation of apoptotic process involved in development [GO:1904747]; is_a positive regulation of reproductive process [GO:2000243]; RO_0002213 nurse cell apoptotic process [GO:0045476] Also known as: up regulation of nurse cell apoptosis, up-regulation of nurse cell apoptosis, upregulation of nurse cell apoptosis, activation of nurse cell apoptosis, positive regulation of nurse cell apoptosis, stimulation of nurse cell apoptosis Sources: GOC:go_curators, GOC:mtg_apoptosis